{
  "gene_symbol": "SOSTDC1",
  "gene_name": "Sclerostin domain-containing protein 1",
  "term_id": "GO:0030514",
  "gene": "UniProtKB:Q6X4U4",
  "term_label": "negative regulation of BMP signaling pathway"
}